{
  "gene_symbol": "GCNT2",
  "gene_name": "N-acetyllactosaminide beta-1,6-N-acetylglucosaminyl-transferase",
  "gene": "UniProtKB:Q8N0V5",
  "term_id": "GO:0008375",
  "term_label": "acetylglucosaminyltransferase activity"
}